{
  "term_label": "positive regulation of neuron projection development",
  "term_id": "GO:0010976",
  "gene_symbol": "DDR1",
  "gene_name": "Epithelial discoidin domain-containing receptor 1",
  "gene": "UniProtKB:Q08345"
}